{
  "gene": "UniProtKB:Q92598",
  "gene_symbol": "HSPH1",
  "term_id": "GO:0005829",
  "term_label": "cytosol",
  "gene_name": "Heat shock protein 105 kDa"
}